{
  "term_label": "monoatomic ion channel complex",
  "term_id": "GO:0034702",
  "gene_symbol": "LRRC8B",
  "gene": "UniProtKB:Q6P9F7",
  "gene_name": "Volume-regulated anion channel subunit LRRC8B"
}